{
  "gene_symbol": "BFAR",
  "gene_name": "Bifunctional apoptosis regulator",
  "gene": "UniProtKB:Q9NZS9",
  "term_label": "ubiquitin protein ligase activity",
  "term_id": "GO:0061630"
}